{
  "gene_symbol": "RRAGD",
  "gene_name": "Ras-related GTP-binding protein D",
  "term_label": "cellular response to starvation",
  "gene": "UniProtKB:Q9NQL2",
  "term_id": "GO:0009267"
}